{
  "gene_name": "RNA guanine-N7 methyltransferase activating subunit",
  "gene": "UniProtKB:Q9BTL3",
  "gene_symbol": "RAMAC",
  "term_label": "mRNA capping enzyme complex",
  "term_id": "GO:0031533"
}